methane biosynthetic process from formic acid [GO:2001127] (biological process) Definition: The chemical reactions and pathways resulting in the formation of a methane from a formic acid. Regulation: regulated by GO:1900339; negatively regulated by negative regulation of methane biosynthetic process from formic acid [GO:1900340]; positively regulated by GO:1900341 Sources: GOC:mengo_curators Relationships: is a type of GO:0015942; is a type of methanogenesis [GO:0015948]